{
  "gene": "UniProtKB:Q8NH18",
  "gene_name": "Olfactory receptor 5J2",
  "gene_symbol": "OR5J2",
  "term_id": "GO:0004984",
  "term_label": "olfactory receptor activity"
}